{
  "gene_symbol": "WNK3",
  "gene": "UniProtKB:Q9BYP7",
  "gene_name": "Serine_threonine-protein kinase WNK3",
  "term_label": "positive regulation of canonical Wnt signaling pathway",
  "term_id": "GO:0090263"
}